{
  "gene_name": "Coiled-coil domain-containing protein 187",
  "term_label": "Unknown molecular function",
  "gene": "UniProtKB:A0A096LP49",
  "gene_symbol": "CCDC187",
  "term_id": "UNKNOWN:0001"
}